{
  "term_label": "cell fate commitment",
  "gene_name": "PR domain zinc finger protein 1",
  "term_id": "GO:0045165",
  "gene_symbol": "PRDM1",
  "gene": "UniProtKB:O75626"
}